xanthosine biosynthetic process [GO:1903229] (biological process) Definition: The chemical reactions and pathways resulting in the formation of xanthosine. References: PMID:7007809, PMID:7559336 Sources: GOC:TermGenie, GO_REF:0000068 Also known as: xanthosine anabolism, xanthosine biosynthesis, xanthosine formation, xanthosine synthesis Relationships: is a type of purine ribonucleoside biosynthetic process [GO:0046129]